detection of pH by carotid body chemoreceptor signaling [GO:0003037] (biological process) Also known as: detection of pH by carotid body chemoreceptor signalling Sources: GOC:mtg_cardio Definition: The process in which information about the levels of hydrogen ions are received and are converted to a molecular signal by chemoreceptors in a carotid body. Relationships: is a type of detection of pH by chemoreceptor signaling [GO:0003022]; is part of detection of hypoxic conditions in blood by carotid body chemoreceptor signaling [GO:0003029]